{
  "gene_name": "VIP36-like protein",
  "gene": "UniProtKB:Q9H0V9",
  "gene_symbol": "LMAN2L",
  "term_id": "GO:0005789",
  "term_label": "endoplasmic reticulum membrane"
}